{
  "term_id": "GO:0005739",
  "gene_name": "Mitochondrial nicotinamide adenine dinucleotide transporter SLC25A51",
  "gene_symbol": "SLC25A51",
  "term_label": "mitochondrion",
  "gene": "UniProtKB:Q9H1U9"
}